{
  "gene": "UniProtKB:O43196",
  "term_label": "double-stranded DNA binding",
  "gene_symbol": "MSH5",
  "gene_name": "MutS protein homolog 5",
  "term_id": "GO:0003690"
}